betaine aldehyde biosynthetic process [GO:1902063] (biological process) Also known as: betaine aldehyde anabolism, betaine aldehyde biosynthesis, betaine aldehyde formation, betaine aldehyde synthesis Definition: The chemical reactions and pathways resulting in the formation of betaine aldehyde. Relationships: is a type of GO:0009058 References: PMID:23563483 Sources: GOC:TermGenie, GOC:di